{
  "term_label": "GTP binding",
  "gene_name": "ADP-ribosylation factor-like protein 14",
  "term_id": "GO:0005525",
  "gene_symbol": "ARL14",
  "gene": "UniProtKB:Q8N4G2"
}